{
  "term_id": "GO:0005886",
  "gene": "UniProtKB:Q8NGS9",
  "gene_symbol": "OR13C2",
  "term_label": "plasma membrane",
  "gene_name": "Olfactory receptor 13C2"
}